{
  "term_id": "UNKNOWN:0001",
  "gene_symbol": "RTL8B",
  "gene": "UniProtKB:Q17RB0",
  "gene_name": "Retrotransposon Gag-like protein 8B",
  "term_label": "Unknown molecular function"
}